{
  "gene_name": "Protein FAM168A",
  "term_id": "UNKNOWN:0003",
  "term_label": "Unknown cellular component",
  "gene": "UniProtKB:Q92567",
  "gene_symbol": "FAM168A"
}